{
  "gene": "UniProtKB:Q9NSY0",
  "gene_symbol": "NRBP2",
  "term_id": "GO:0090263",
  "term_label": "positive regulation of canonical Wnt signaling pathway",
  "gene_name": "Nuclear receptor-binding protein 2"
}